{
  "term_label": "synapse assembly",
  "gene_symbol": "PLXNA3",
  "gene_name": "Plexin-A3",
  "gene": "UniProtKB:P51805",
  "term_id": "GO:0007416"
}